{
  "term_id": "UNKNOWN:0002",
  "gene_symbol": "KRTAP21-3",
  "gene": "UniProtKB:Q3LHN1",
  "term_label": "Unknown biological process",
  "gene_name": "Keratin-associated protein 21-3"
}